negative regulation of ribosomal subunit export from nucleus [GO:2000201] (biological process) Subtypes: negative regulation of ribosomal large subunit export from nucleus [GO:2000204], negative regulation of ribosomal small subunit export from nucleus [GO:2000207] Also known as: negative regulation of ribosomal subunit export from cell nucleus, negative regulation of ribosomal subunit export out of nucleus, negative regulation of ribosomal subunit transport from nucleus to cytoplasm, negative regulation of ribosomal subunit-nucleus export, negative regulation of ribosome export from nucleus Relationships: is a type of negative regulation of nucleocytoplasmic transport [GO:0046823]; is_a negative regulation of ribosome biogenesis [GO:0090071]; is a type of negative regulation of ribonucleoprotein complex localization [GO:2000198]; is a type of regulation of ribosomal subunit export from nucleus [GO:2000200]; negatively regulates ribosomal subunit export from nucleus [GO:0000054] Definition: Any process that stops, prevents, or reduces the frequency, rate or extent of ribosomal subunit export from nucleus. Sources: GOC:mah